{
  "term_id": "GO:0000159",
  "gene": "UniProtKB:P30154",
  "gene_symbol": "PPP2R1B",
  "term_label": "protein phosphatase type 2A complex",
  "gene_name": "Serine_threonine-protein phosphatase 2A 65 kDa regulatory subunit A beta isoform"
}